{
  "gene_symbol": "WHRN",
  "gene": "UniProtKB:Q9P202",
  "gene_name": "Whirlin",
  "term_id": "GO:0032426",
  "term_label": "stereocilium tip"
}